{
  "gene_name": "E3 ubiquitin-protein ligase RNF167",
  "term_label": "ubiquitin-dependent protein catabolic process",
  "gene_symbol": "RNF167",
  "term_id": "GO:0006511",
  "gene": "UniProtKB:Q9H6Y7"
}